{
  "term_label": "G protein-coupled receptor signaling pathway",
  "gene": "UniProtKB:Q9H1Y3",
  "gene_name": "Opsin-3",
  "term_id": "GO:0007186",
  "gene_symbol": "OPN3"
}